subplasmalemmal coating [GO:0044280] (cellular component) Definition: Electron dense material observed coating the cytoplasmic face of the plasma membrane in certain regions of a neuron, e.g., the axon initial segment; the nodal membrane at the Node of Ranvier. Sources: NIF_Subcellular:sao1938587839 Relationships: is_a cellular anatomical structure [GO:0110165]; is part of GO:0031234